{
  "term_label": "cytokine receptor binding",
  "gene_name": "Suppressor of cytokine signaling 2",
  "gene_symbol": "SOCS2",
  "term_id": "GO:0005126",
  "gene": "UniProtKB:O14508"
}